{
  "gene_symbol": "LGI1",
  "gene": "UniProtKB:O95970",
  "gene_name": "Leucine-rich glioma-inactivated protein 1",
  "term_id": "UNKNOWN:0002",
  "term_label": "Unknown biological process"
}